all-trans-retinol 13,14-reductase activity [GO:0051786] (molecular function) Also known as: (13,14)-all-trans-retinol saturase activity, all-trans-13,14-dihydroretinol:acceptor 13,14-oxidoreductase activity, all-trans-retinol:all-trans-13,14-dihydroretinol saturase activity, RetSat activity, retinol saturase activity Relationships: is a type of oxidoreductase activity, acting on the CH-CH group of donors [GO:0016627]; is part of GO:0042572 Sources: EC:1.3.99.23, RHEA:19193 Definition: Catalysis of the reaction: all-trans-13,14-dihydroretinol + A = all-trans-retinol + AH(2). Note that this reaction has only been observed to occur in the opposite direction.